{
  "gene": "UniProtKB:Q6ZW61",
  "term_label": "photoreceptor cell maintenance",
  "gene_name": "Bardet-Biedl syndrome 12 protein",
  "gene_symbol": "BBS12",
  "term_id": "GO:0045494"
}